{
  "term_label": "malonyl-CoA catabolic process",
  "gene_symbol": "MLYCD",
  "gene": "UniProtKB:O95822",
  "gene_name": "Malonyl-CoA decarboxylase, mitochondrial",
  "term_id": "GO:2001294"
}